negative regulation of complement activation, lectin pathway [GO:0001869] (biological process) Relationships: is a type of regulation of complement activation, lectin pathway [GO:0001868]; is a type of GO:0045824; is_a negative regulation of complement activation [GO:0045916]; negatively regulates complement activation, lectin pathway [GO:0001867] Sources: GOC:add, ISBN:0781735149 Also known as: down regulation of complement activation, lectin pathway, down-regulation of complement activation, lectin pathway, downregulation of complement activation, lectin pathway, negative regulation of complement cascade, lectin pathway, inhibition of complement activation, lectin pathway Definition: Any process that stops, prevents, or reduces the rate of complement activation by the lectin pathway.